{
  "gene": "UniProtKB:Q7Z406",
  "term_id": "GO:0008360",
  "gene_symbol": "MYH14",
  "term_label": "regulation of cell shape",
  "gene_name": "Myosin-14"
}